{
  "gene_symbol": "PEX5",
  "gene_name": "Peroxisomal targeting signal 1 receptor",
  "term_label": "cytosol",
  "term_id": "GO:0005829",
  "gene": "UniProtKB:P50542"
}